{
  "gene": "UniProtKB:P28838",
  "gene_name": "Cytosol aminopeptidase",
  "term_label": "proteolysis",
  "term_id": "GO:0006508",
  "gene_symbol": "LAP3"
}